{
  "term_id": "GO:0035556",
  "gene": "UniProtKB:Q9UHY1",
  "gene_name": "Nuclear receptor-binding protein",
  "term_label": "intracellular signal transduction",
  "gene_symbol": "NRBP1"
}